{
  "gene_name": "F-box only protein 10",
  "gene_symbol": "FBXO10",
  "term_label": "Unknown cellular component",
  "gene": "UniProtKB:Q9UK96",
  "term_id": "UNKNOWN:0003"
}